protein farnesyltransferase activity [GO:0004660] (molecular function) References: PMID:8621375 Sources: RHEA:13345 Also known as: protein-cysteine farnesyltransferase activity, CAAX farnesyltransferase activity, FTase activity, farnesyl-diphosphate:protein-cysteine farnesyltransferase activity Note: The catalyzed reaction transfers a farnesyl group from farnesyl diphosphate to a target protein. There is no relationship between this activity and farnesyltransferase activity, GO:0004311, where the catalyzed reaction forms (free) geranylgeranyl diphosphate. Relationships: is a type of protein prenyltransferase activity [GO:0008318] Definition: Catalysis of the reaction: L-cysteinyl-[protein] + (2E,6E)-farnesyl diphosphate = S-(2E,6E)-farnesyl-L-cysteinyl-[protein] + diphosphate.